{
  "term_id": "GO:0031410",
  "gene_name": "NEDD4-binding protein 3",
  "gene": "UniProtKB:O15049",
  "gene_symbol": "N4BP3",
  "term_label": "cytoplasmic vesicle"
}